{
  "term_id": "GO:0015629",
  "gene": "UniProtKB:O94832",
  "term_label": "actin cytoskeleton",
  "gene_name": "Unconventional myosin-Id",
  "gene_symbol": "MYO1D"
}